{
  "gene": "UniProtKB:Q6DT37",
  "term_id": "GO:0005737",
  "gene_name": "Serine_threonine-protein kinase MRCK gamma",
  "gene_symbol": "CDC42BPG",
  "term_label": "cytoplasm"
}